cellular response to zinc ion starvation [GO:0034224] (biological process) Also known as: cellular response to zinc ion limitation, cellular response to zinc starvation Sources: GOC:mah Relationships: is a type of cellular response to starvation [GO:0009267]; is a type of response to zinc ion starvation [GO:0120127] Definition: Any process that results in a change in state or activity of a cell (in terms of movement, secretion, enzyme production, gene expression, etc.) as a result of deprivation of zinc ions.